{
  "gene_name": "DBF4-type zinc finger-containing protein 2",
  "gene_symbol": "ZDBF2",
  "term_label": "Unknown cellular component",
  "term_id": "UNKNOWN:0003",
  "gene": "UniProtKB:Q9HCK1"
}